poly-N-acetyllactosamine biosynthetic process [GO:0030311] (biological process) Definition: The chemical reactions and pathways resulting in the formation of poly-N-acetyllactosamine, a carbohydrate composed of N-acetyllactosamine repeats (Gal-beta-1,4-GlcNAc-beta-1,3)n. Relationships: is a type of aminoglycan biosynthetic process [GO:0006023]; is a type of GO:0030309 References: PMID:9405606 Sources: GOC:mah Also known as: poly-N-acetyllactosamine anabolism, poly-N-acetyllactosamine biosynthesis, poly-N-acetyllactosamine formation, poly-N-acetyllactosamine synthesis